bone mineralization [GO:0030282] (biological process) Also known as: bone calcification Regulation: RO_0002211 by regulation of bone mineralization [GO:0030500]; positively regulated by positive regulation of bone mineralization [GO:0030501]; negatively regulated by negative regulation of bone mineralization [GO:0030502] Subtypes: bone mineralization involved in bone maturation [GO:0035630] Relationships: is a type of biomineral tissue development [GO:0031214]; is part of ossification [GO:0001503] Definition: The deposition of hydroxyapatite, a form of calcium phosphate with the formula Ca10(PO4)6(OH)2, in bone tissue. References: PMID:22936354 Sources: GOC:mah